{
  "term_label": "Unknown cellular component",
  "gene_name": "Carbohydrate sulfotransferase 13",
  "gene_symbol": "CHST13",
  "term_id": "UNKNOWN:0003",
  "gene": "UniProtKB:Q8NET6"
}